response to diacyl bacterial lipopeptide [GO:0071724] (biological process) Definition: Any process that results in a change in state or activity of a cell or an organism (in terms of movement, secretion, enzyme production, gene expression, etc.) as a result of a diacylated bacterial lipopeptide stimulus. Relationships: is a type of response to bacterial lipopeptide [GO:0070339] Subtypes: detection of diacyl bacterial lipopeptide [GO:0042496], cellular response to diacyl bacterial lipopeptide [GO:0071726] References: PMID:12077222, PMID:12524386, PMID:2757794 Sources: GOC:add Also known as: response to diacylated bacterial lipoprotein Note: Note that bacterial lipopeptides are derived from bacterial lipoproteins, but the two terms are sometimes used interchangeably in the literature.